{
  "term_label": "response to peptide hormone",
  "term_id": "GO:0043434",
  "gene_name": "Signal transducer and activator of transcription 5A",
  "gene": "UniProtKB:P42229",
  "gene_symbol": "STAT5A"
}